{
  "term_label": "mRNA binding",
  "term_id": "GO:0003729",
  "gene_name": "U6 snRNA-associated Sm-like protein LSm1",
  "gene": "UniProtKB:O15116",
  "gene_symbol": "LSM1"
}